{
  "gene": "UniProtKB:Q13023",
  "term_label": "nuclear membrane",
  "gene_symbol": "AKAP6",
  "term_id": "GO:0031965",
  "gene_name": "A-kinase anchor protein 6"
}